{
  "gene_name": "Y-box-binding protein 1",
  "term_label": "nucleus",
  "term_id": "GO:0005634",
  "gene_symbol": "YBX1",
  "gene": "UniProtKB:P67809"
}